{
  "term_id": "UNKNOWN:0003",
  "gene": "UniProtKB:Q5T5A4",
  "gene_name": "Cilia- and flagella-associated protein 276",
  "term_label": "Unknown cellular component",
  "gene_symbol": "CFAP276"
}